{
  "gene": "UniProtKB:Q86UQ4",
  "term_id": "UNKNOWN:0003",
  "gene_symbol": "ABCA13",
  "gene_name": "ATP-binding cassette sub-family A member 13",
  "term_label": "Unknown cellular component"
}